{
  "gene": "UniProtKB:Q8NHS1",
  "gene_symbol": "CLDND2",
  "term_id": "GO:0005886",
  "gene_name": "Claudin domain-containing protein 2",
  "term_label": "plasma membrane"
}